{
  "term_label": "negative regulation of stress fiber assembly",
  "gene_name": "Rho GTPase-activating protein 28",
  "term_id": "GO:0051497",
  "gene": "UniProtKB:Q9P2N2",
  "gene_symbol": "ARHGAP28"
}